{
  "gene_symbol": "SDHA",
  "gene": "UniProtKB:P31040",
  "gene_name": "Succinate dehydrogenase [ubiquinone] flavoprotein subunit, mitochondrial",
  "term_id": "GO:0050660",
  "term_label": "flavin adenine dinucleotide binding"
}